imaginal disc-derived leg segmentation [GO:0036011] (BP) Definition: Division of an imaginal disc-derived leg into a series of semi-repetitive parts or segments. The Drosophila leg, for example, has nine segments, each separated from the next by a flexible joint. Relationships: is a type of appendage segmentation [GO:0035285]; is part of imaginal disc-derived leg morphogenesis [GO:0007480] Sources: GOC:bf